nuclear division [GO:0000280] (biological process) Also known as: karyokinesis Relationships: is a type of organelle fission [GO:0048285] Regulation: regulated by regulation of nuclear division [GO:0051783]; negatively regulated by GO:0051784; positively regulated by positive regulation of nuclear division [GO:0051785] Sources: GOC:mah Subtypes: amitosis [GO:0051337], meiotic nuclear division [GO:0140013], mitotic nuclear division [GO:0140014] Definition: The division of a cell nucleus into two nuclei, with DNA and other nuclear contents distributed between the daughter nuclei.